{
  "term_label": "protein-membrane adaptor activity",
  "gene": "UniProtKB:Q96JE7",
  "gene_name": "Protein transport protein Sec16B",
  "gene_symbol": "SEC16B",
  "term_id": "GO:0043495"
}